{
  "gene_name": "Protein FAM27E3",
  "gene": "UniProtKB:Q08E93",
  "gene_symbol": "FAM27E3",
  "term_label": "Unknown molecular function",
  "term_id": "UNKNOWN:0001"
}